{
  "term_label": "GARP complex",
  "term_id": "GO:0000938",
  "gene_symbol": "VPS54",
  "gene": "UniProtKB:Q9P1Q0",
  "gene_name": "Vacuolar protein sorting-associated protein 54"
}